{
  "gene_name": "WD repeat-containing protein 81",
  "gene": "UniProtKB:Q562E7",
  "gene_symbol": "WDR81",
  "term_label": "aggrephagy",
  "term_id": "GO:0035973"
}